{
  "gene": "UniProtKB:A8MUV8",
  "term_label": "Unknown cellular component",
  "gene_name": "Putative zinc finger protein 727",
  "term_id": "UNKNOWN:0003",
  "gene_symbol": "ZNF727"
}